{
  "gene_symbol": "ELAVL2",
  "gene": "UniProtKB:Q12926",
  "gene_name": "ELAV-like protein 2",
  "term_label": "protein-RNA adaptor activity",
  "term_id": "GO:0140517"
}